{
  "gene": "UniProtKB:O43908",
  "term_label": "natural killer cell mediated immunity",
  "gene_symbol": "KLRC4",
  "gene_name": "NKG2-F type II integral membrane protein",
  "term_id": "GO:0002228"
}